{
  "term_label": "U4/U6 x U5 tri-snRNP complex",
  "gene_name": "Pre-mRNA-processing factor 6",
  "gene": "UniProtKB:O94906",
  "gene_symbol": "PRPF6",
  "term_id": "GO:0046540"
}